L-arginine catabolic process to proline via ornithine [GO:0010121] (biological process) Definition: The chemical reactions and pathways resulting in the breakdown of arginine into other compounds, including proline, via ornithine. Also known as: arginine breakdown to proline via ornithine, arginine degradation to proline via ornithine Relationships: is a type of L-arginine catabolic process to L-proline [GO:0019493] Sources: GOC:pz